{
  "gene_name": "NF-X1-type zinc finger protein NFXL1",
  "gene": "UniProtKB:Q6ZNB6",
  "term_label": "DNA-binding transcription factor activity, RNA polymerase II-specific",
  "gene_symbol": "NFXL1",
  "term_id": "GO:0000981"
}